{
  "gene_symbol": "CARD10",
  "gene": "UniProtKB:Q9BWT7",
  "gene_name": "Caspase recruitment domain-containing protein 10",
  "term_label": "signaling adaptor activity",
  "term_id": "GO:0035591"
}